protein peptidyl-prolyl isomerization [GO:0000413] (biological process) Definition: The modification of a protein by cis-trans isomerization of a proline residue. References: PMID:16959570 Sources: GOC:krc Also known as: protein proline isomerization Relationships: is a type of peptidyl-proline modification [GO:0018208]